{
  "gene_name": "R3H domain-containing protein 2",
  "term_id": "UNKNOWN:0001",
  "gene": "UniProtKB:Q9Y2K5",
  "term_label": "Unknown molecular function",
  "gene_symbol": "R3HDM2"
}